{
  "gene_symbol": "MAGED1",
  "term_id": "UNKNOWN:0001",
  "gene": "UniProtKB:Q9Y5V3",
  "gene_name": "Melanoma-associated antigen D1",
  "term_label": "Unknown molecular function"
}